{
  "term_label": "endoplasmic reticulum membrane",
  "term_id": "GO:0005789",
  "gene_name": "E3 ubiquitin-protein ligase RNF180",
  "gene": "UniProtKB:Q86T96",
  "gene_symbol": "RNF180"
}